{
  "gene": "UniProtKB:Q8IY33",
  "term_label": "actin filament binding",
  "term_id": "GO:0051015",
  "gene_name": "MICAL-like protein 2",
  "gene_symbol": "MICALL2"
}